{
  "gene": "UniProtKB:Q9Y5X3",
  "term_id": "GO:0006907",
  "gene_name": "Sorting nexin-5",
  "term_label": "pinocytosis",
  "gene_symbol": "SNX5"
}